{
  "term_label": "immunoglobulin complex",
  "gene_name": "Immunoglobulin kappa variable 2D-40",
  "gene_symbol": "IGKV2D-40",
  "term_id": "GO:0019814",
  "gene": "UniProtKB:P01614"
}